{
  "gene": "UniProtKB:O00421",
  "term_id": "GO:0005737",
  "gene_symbol": "CCRL2",
  "gene_name": "C-C chemokine receptor-like 2",
  "term_label": "cytoplasm"
}